{
  "gene_name": "A-kinase anchor protein 5",
  "term_id": "GO:0008179",
  "term_label": "adenylate cyclase binding",
  "gene_symbol": "AKAP5",
  "gene": "UniProtKB:P24588"
}